{
  "gene_symbol": "PDGFB",
  "gene": "UniProtKB:P01127",
  "term_label": "platelet-derived growth factor receptor signaling pathway",
  "gene_name": "Platelet-derived growth factor subunit B",
  "term_id": "GO:0048008"
}